{
  "term_label": "cytoskeleton",
  "gene": "UniProtKB:O76015",
  "term_id": "GO:0005856",
  "gene_symbol": "KRT38",
  "gene_name": "Keratin, type I cuticular Ha8"
}